{
  "gene_name": "POTE ankyrin domain family member I",
  "term_id": "GO:0030424",
  "gene": "UniProtKB:P0CG38",
  "gene_symbol": "POTEI",
  "term_label": "axon"
}